glomerulus vasculature morphogenesis [GO:0072103] (biological process) Sources: GOC:mtg_kidney_jan10 Definition: The process in which the anatomical structures of the glomerulus vasculature are generated and organized. The glomerulus vasculature is composed of the tubule structures that carry blood or lymph in the glomerulus. Subtypes: mesonephric glomerulus vasculature morphogenesis [GO:0061248], GO:0072276 Relationships: is a type of blood vessel morphogenesis [GO:0048514]; is a type of kidney vasculature morphogenesis [GO:0061439]; is part of GO:0072012; is part of GO:0072102